{
  "term_id": "GO:0006457",
  "gene": "UniProtKB:Q8N4E4",
  "term_label": "protein folding",
  "gene_name": "Phosducin-like protein 2",
  "gene_symbol": "PDCL2"
}